{
  "term_id": "GO:0045786",
  "term_label": "negative regulation of cell cycle",
  "gene_name": "Nuclear protein 2",
  "gene_symbol": "NUPR2",
  "gene": "UniProtKB:A6NF83"
}